{
  "gene": "UniProtKB:Q14721",
  "term_label": "dendrite membrane",
  "gene_symbol": "KCNB1",
  "term_id": "GO:0032590",
  "gene_name": "Potassium voltage-gated channel subfamily B member 1"
}